{
  "term_id": "GO:0000978",
  "gene_name": "Pituitary homeobox 1",
  "gene_symbol": "PITX1",
  "gene": "UniProtKB:P78337",
  "term_label": "RNA polymerase II cis-regulatory region sequence-specific DNA binding"
}